coenzyme F420-dependent N5,N10-methenyltetrahydromethanopterin reductase activity [GO:0018537] (molecular function) Sources: EC:1.5.98.2, RHEA:21144 Definition: Catalysis of the reaction: 5-methyltetrahydromethanopterin + coenzyme F420 + H+ = 5,10-methylenetetrahydromethanopterin + reduced coenzyme F420. Relationships: is a type of oxidoreductase activity, acting on the CH-NH group of donors [GO:0016645] Also known as: methylenetetrahydromethanopterin reductase activity, 5,10-methylenetetrahydromethanopterin cyclohydrolase activity, 5,10-methylenetetrahydromethanopterin reductase activity, 5-methyltetrahydromethanopterin:coenzyme-F420 oxidoreductase activity, N(5),N(10)-methylenetetrahydromethanopterin reductase activity, N(5),N(10)-methylenetetrahydromethanopterin:coenzyme-F420 oxidoreductase activity, N5,N10-methylenetetrahydromethanopterin reductase activity, N5,N10-methylenetetrahydromethanopterin:coenzyme-F420 oxidoreductase activity, coenzyme F420-dependent N(5),N(10)-methenyltetrahydromethanopterin reductase activity, methylene-H(4)MPT reductase activity, methylene-H4MPT reductase activity